presynapse organization [GO:0099172] (biological process) Subtypes: terminal button organization [GO:0072553], presynapse assembly [GO:0099054] Also known as: presynapse development, presynapse organisation, presynapse morphogenesis, presynapse organization and biogenesis Regulation: regulated by GO:0099174 Definition: A process that is carried out at the cellular level which results in the assembly, arrangement of constituent parts, or disassembly of a presynapse. Relationships: is a type of cellular component organization [GO:0016043]; is part of synapse organization [GO:0050808] Sources: GOC:dos